{
  "gene_name": "DnaJ homolog subfamily B member 3",
  "gene_symbol": "DNAJB3",
  "term_id": "UNKNOWN:0002",
  "gene": "UniProtKB:Q8WWF6",
  "term_label": "Unknown biological process"
}